{
  "gene_name": "rRNA-processing protein FCF1 homolog",
  "term_label": "nucleolus",
  "gene_symbol": "FCF1",
  "gene": "UniProtKB:Q9Y324",
  "term_id": "GO:0005730"
}